{
  "term_id": "GO:0004065",
  "gene_name": "Arylsulfatase D",
  "gene_symbol": "ARSD",
  "term_label": "arylsulfatase activity",
  "gene": "UniProtKB:P51689"
}